deoxylimonate A-ring-lactonase activity [GO:0047845] (molecular function) Also known as: deoxylimonate A-ring-lactonohydrolase activity Sources: EC:3.1.1.46, RHEA:14997 Definition: Catalysis of the reaction: deoxylimonoate + H2O = deoxylimononate D-ring-lactone + H+. Relationships: is_a carboxylic ester hydrolase activity [GO:0052689]